{
  "term_id": "GO:0005886",
  "gene_name": "Semaphorin-6B",
  "term_label": "plasma membrane",
  "gene": "UniProtKB:Q9H3T3",
  "gene_symbol": "SEMA6B"
}